{
  "term_id": "GO:0005802",
  "term_label": "trans-Golgi network",
  "gene_name": "Carbohydrate sulfotransferase 2",
  "gene": "UniProtKB:Q9Y4C5",
  "gene_symbol": "CHST2"
}